{
  "term_label": "intrinsic apoptotic signaling pathway in response to DNA damage",
  "gene": "UniProtKB:Q9UMX3",
  "term_id": "GO:0008630",
  "gene_name": "Bcl-2-related ovarian killer protein",
  "gene_symbol": "BOK"
}